{
  "term_id": "GO:0005886",
  "gene": "UniProtKB:O14924",
  "gene_symbol": "RGS12",
  "gene_name": "Regulator of G-protein signaling 12",
  "term_label": "plasma membrane"
}